heart growth [GO:0060419] (biological process) Sources: GOC:dph, GOC:tb Definition: The increase in size or mass of the heart. Regulation: regulated by regulation of heart growth [GO:0060420]; positively regulated by GO:0060421; negatively regulated by negative regulation of heart growth [GO:0061117] Relationships: is a type of organ growth [GO:0035265]; is part of GO:0007507